{
  "gene_name": "Protein FAM98B",
  "gene": "UniProtKB:Q52LJ0",
  "gene_symbol": "FAM98B",
  "term_id": "UNKNOWN:0001",
  "term_label": "Unknown molecular function"
}